{
  "gene_name": "Phakinin",
  "term_label": "Unknown molecular function",
  "gene": "UniProtKB:Q13515",
  "gene_symbol": "BFSP2",
  "term_id": "UNKNOWN:0001"
}